{
  "gene_symbol": "ZNF500",
  "gene_name": "Zinc finger protein 500",
  "term_label": "regulation of transcription by RNA polymerase II",
  "term_id": "GO:0006357",
  "gene": "UniProtKB:O60304"
}